regulation of secretion of lysosomal enzymes [GO:0090182] (biological process) Definition: Any process that modulates the rate, frequency or extent of secretion of lysosomal enzymes, the controlled release of lysosomal enzymes by a cell. Sources: GOC:BHF, GOC:dph, GOC:tb Relationships: is a type of regulation of protein secretion [GO:0050708]; regulates secretion of lysosomal enzymes [GO:0033299] Subtypes: positive regulation of secretion of lysosomal enzymes [GO:0090340], negative regulation of secretion of lysosomal enzymes [GO:0090341]